superoxide-generating NADPH oxidase activator activity [GO:0016176] (molecular function) Sources: GOC:ai Relationships: is a type of enzyme activator activity [GO:0008047]; positively regulates GO:0106292 Also known as: neutrophil cytosol factor 2 Definition: Binds to and increases the activity of the enzyme superoxide-generating NADPH oxidase.